{
  "gene": "UniProtKB:Q5VXT5",
  "term_label": "Unknown biological process",
  "term_id": "UNKNOWN:0002",
  "gene_symbol": "SYPL2",
  "gene_name": "Synaptophysin-like protein 2"
}